{
  "term_id": "GO:0007409",
  "gene_name": "Cyclin-dependent kinase 5",
  "term_label": "axonogenesis",
  "gene_symbol": "CDK5",
  "gene": "UniProtKB:Q00535"
}